{
  "gene_name": "Procollagen-lysine,2-oxoglutarate 5-dioxygenase 2",
  "gene_symbol": "PLOD2",
  "gene": "UniProtKB:O00469",
  "term_label": "procollagen-lysine 5-dioxygenase activity",
  "term_id": "GO:0008475"
}